{
  "gene": "UniProtKB:Q8TAA9",
  "gene_symbol": "VANGL1",
  "gene_name": "Vang-like protein 1",
  "term_id": "UNKNOWN:0002",
  "term_label": "Unknown biological process"
}